{
  "term_label": "Unknown cellular component",
  "gene_symbol": "CT45A9",
  "term_id": "UNKNOWN:0003",
  "gene": "UniProtKB:P0DMV2",
  "gene_name": "Cancer_testis antigen family 45 member A9"
}